{
  "gene": "UniProtKB:P35070",
  "gene_name": "Probetacellulin",
  "term_label": "growth factor activity",
  "gene_symbol": "BTC",
  "term_id": "GO:0008083"
}